{
  "term_id": "GO:0000978",
  "gene": "UniProtKB:P49716",
  "gene_symbol": "CEBPD",
  "gene_name": "CCAAT_enhancer-binding protein delta",
  "term_label": "RNA polymerase II cis-regulatory region sequence-specific DNA binding"
}